{
  "term_id": "GO:0070059",
  "term_label": "intrinsic apoptotic signaling pathway in response to endoplasmic reticulum stress",
  "gene_symbol": "BBC3",
  "gene": "UniProtKB:Q96PG8",
  "gene_name": "Bcl-2-binding component 3, isoforms 3_4"
}